{
  "gene_name": "SH2 domain-containing adapter protein D",
  "term_id": "GO:0001784",
  "term_label": "phosphotyrosine residue binding",
  "gene": "UniProtKB:Q96IW2",
  "gene_symbol": "SHD"
}